{
  "gene_symbol": "FCRL2",
  "gene_name": "Fc receptor-like protein 2",
  "term_label": "external side of plasma membrane",
  "term_id": "GO:0009897",
  "gene": "UniProtKB:Q96LA5"
}